pullulan metabolic process [GO:0051676] (biological process) Subtypes: pullulan biosynthetic process [GO:0051677], pullulan catabolic process [GO:0051678] Definition: The chemical reactions and pathways involving pullulan, a neutral linear polysaccharide composed of repeating units of maltotriose joined by alpha-(1,6)-linkages. References: PMID:15013381 Relationships: is_a glucan metabolic process [GO:0044042] Also known as: pullulan metabolism